{
  "term_label": "protein exit from endoplasmic reticulum",
  "term_id": "GO:0032527",
  "gene_symbol": "TECPR2",
  "gene_name": "Tectonin beta-propeller repeat-containing protein 2",
  "gene": "UniProtKB:O15040"
}